{
  "term_label": "RNA polymerase III complex",
  "gene_symbol": "POLR1C",
  "gene": "UniProtKB:O15160",
  "term_id": "GO:0005666",
  "gene_name": "DNA-directed RNA polymerases I and III subunit RPAC1"
}